{
  "gene_symbol": "HRH1",
  "term_label": "chemical synaptic transmission",
  "term_id": "GO:0007268",
  "gene_name": "Histamine H1 receptor",
  "gene": "UniProtKB:P35367"
}